{
  "gene_symbol": "KRTAP4-8",
  "term_label": "Unknown cellular component",
  "gene": "UniProtKB:A0A0G2JLE6",
  "term_id": "UNKNOWN:0003",
  "gene_name": "HCG2042992"
}